negative regulation of T cell activation via T cell receptor contact with antigen bound to MHC molecule on antigen presenting cell [GO:2001189] (biological process) Relationships: is a type of negative regulation of immune effector process [GO:0002698]; is a type of negative regulation of immune response [GO:0050777]; is a type of GO:0050868; is a type of regulation of T cell activation via T cell receptor contact with antigen bound to MHC molecule on antigen presenting cell [GO:2001188]; RO_0002212 T cell activation via T cell receptor contact with antigen bound to MHC molecule on antigen presenting cell [GO:0002291] Definition: Any process that stops, prevents or reduces the frequency, rate or extent of T cell activation via T cell receptor contact with antigen bound to MHC molecule on antigen presenting cell. Also known as: negative regulation of T lymphocyte activation via T cell receptor contact with antigen bound to MHC molecule on antigen presenting cell, negative regulation of T-cell activation via T cell receptor contact with antigen bound to MHC molecule on antigen presenting cell, negative regulation of T-lymphocyte activation via T cell receptor contact with antigen bound to MHC molecule on antigen presenting cell Sources: GOC:obol